{
  "gene": "UniProtKB:Q96LW4",
  "gene_name": "DNA-directed primase_polymerase protein",
  "term_id": "GO:0006264",
  "gene_symbol": "PRIMPOL",
  "term_label": "mitochondrial DNA replication"
}